{
  "term_label": "intermediate filament cytoskeleton organization",
  "gene_symbol": "DSP",
  "gene": "UniProtKB:P15924",
  "gene_name": "Desmoplakin",
  "term_id": "GO:0045104"
}